{
  "term_label": "Unknown cellular component",
  "gene_name": "Heparan-sulfate 6-O-sulfotransferase 1",
  "gene_symbol": "HS6ST1",
  "gene": "UniProtKB:O60243",
  "term_id": "UNKNOWN:0003"
}